histone H2AXY142 phosphatase activity [GO:0140793] (molecular function) Relationships: is a type of GO:0140789 Also known as: histone H2-Y142 phosphatase activity, histone tyrosine phosphatase activity (H2-Y142 specific), histone H2Y142 phosphatase activity References: PMID:19234442, PMID:19351884 Note: Note that the residue position corresponds to the canonical human H2AX histone (UniProtKB:P16104); this residue is conserved in mammals, but missing from tetrahymena. This residue is present in Drosophila histone H2AV. Residue 1 is the first residue following removal of the initiating Methionine (Met). Note that each histone is encoded by multiple genes, and sequences may vary across different genes within an organism. Definition: Catalysis of the reaction: histone H2AX tyrosine phosphate (position 142) + H2O = histone H2AX tyrosine (position 142) + phosphate.